{
  "gene": "UniProtKB:Q9ULB1",
  "gene_symbol": "NRXN1",
  "term_id": "GO:0007165",
  "term_label": "signal transduction",
  "gene_name": "Neurexin-1"
}